{
  "term_label": "brain development",
  "gene_symbol": "CNTN5",
  "term_id": "GO:0007420",
  "gene_name": "Contactin-5",
  "gene": "UniProtKB:O94779"
}